glycerophospholipid catabolic process [GO:0046475] (biological process) Relationships: is a type of glycerophospholipid metabolic process [GO:0006650]; is a type of phospholipid catabolic process [GO:0009395]; is a type of glycerolipid catabolic process [GO:0046503] Also known as: glycerophospholipid breakdown, glycerophospholipid catabolism, glycerophospholipid degradation, phosphoglyceride catabolic process, phosphoglyceride catabolism Subtypes: phosphatidylserine catabolic process [GO:0006660], phosphatidylinositol catabolic process [GO:0031161], phosphatidylglycerol catabolic process [GO:0034478], phosphatidylcholine catabolic process [GO:0034638], phosphatidylethanolamine catabolic process [GO:0046338], CDP-diacylglycerol catabolic process [GO:0046342], platelet activating factor catabolic process [GO:0062234] Definition: The chemical reactions and pathways resulting in the breakdown of glycerophospholipids, any derivative of glycerophosphate that contains at least one O-acyl, O-alkyl, or O-alkenyl group attached to the glycerol residue. Sources: ISBN:0198506732